{
  "term_id": "UNKNOWN:0001",
  "gene": "UniProtKB:Q8IYH5",
  "term_label": "Unknown molecular function",
  "gene_symbol": "ZZZ3",
  "gene_name": "ZZ-type zinc finger-containing protein 3"
}